{
  "gene_symbol": "PAK6-AS1",
  "gene": "UniProtKB:Q8N910",
  "term_label": "Unknown cellular component",
  "gene_name": "Putative uncharacterized protein PAK6-AS1",
  "term_id": "UNKNOWN:0003"
}